{
  "gene_name": "Lysosomal-trafficking regulator",
  "gene": "UniProtKB:Q99698",
  "gene_symbol": "LYST",
  "term_id": "UNKNOWN:0001",
  "term_label": "Unknown molecular function"
}